negative regulation of phospholipid metabolic process [GO:1903726] (biological process) Definition: Any process that stops, prevents or reduces the frequency, rate or extent of phospholipid metabolic process. Also known as: down regulation of phospholipid metabolic process, down regulation of phospholipid metabolism, down-regulation of phospholipid metabolic process, down-regulation of phospholipid metabolism, downregulation of phospholipid metabolic process, downregulation of phospholipid metabolism, negative regulation of phospholipid metabolism, inhibition of phospholipid metabolic process, inhibition of phospholipid metabolism References: PMID:10657240 Sources: GOC:TermGenie, GO_REF:0000058 Subtypes: negative regulation of phosphatidylcholine catabolic process [GO:0010900], GO:0071072, negative regulation of cardiolipin metabolic process [GO:1900209], negative regulation of 1-phosphatidyl-1D-myo-inositol 4,5-bisphosphate catabolic process [GO:1902642] Relationships: is a type of negative regulation of lipid metabolic process [GO:0045833]; is a type of GO:0045936; is a type of regulation of phospholipid metabolic process [GO:1903725]; negatively regulates phospholipid metabolic process [GO:0006644]